{
  "term_id": "GO:0005634",
  "gene_symbol": "TACSTD2",
  "gene_name": "Tumor-associated calcium signal transducer 2",
  "gene": "UniProtKB:P09758",
  "term_label": "nucleus"
}